regulation of protein import [GO:1904589] (biological process) Also known as: regulation of protein uptake Definition: Any process that modulates the frequency, rate or extent of protein import. References: PMID:11406629 Sources: GOC:TermGenie, GO_REF:0000058 Relationships: is a type of regulation of protein transport [GO:0051223]; regulates protein import [GO:0017038] Subtypes: GO:1904590, GO:1904591